detection of protozoan [GO:0001563] (biological process) Sources: GOC:ai Also known as: detection of protozoa, detection of protozoon, perception of protozoa Definition: The series of events in which a stimulus from a protozoan is received and converted into a molecular signal. Relationships: is_a GO:0001562; is a type of detection of other organism [GO:0098543]